galactose transmembrane transport [GO:0015757] (biological process) Definition: The process in which galactose is transported across a lipid bilayer, from one side of a membrane to the other. D-galactose is widely distributed in combined form in plants, animals and microorganisms as a constituent of oligo- and polysaccharides; it also occurs in galactolipids and as its glucoside in lactose and melibiose. Relationships: is a type of hexose transmembrane transport [GO:0008645] Sources: GOC:ai Subtypes: GO:0140425 Also known as: galactose transport